{
  "gene_name": "Calmodulin-regulated spectrin-associated protein 3",
  "gene": "UniProtKB:Q9P1Y5",
  "gene_symbol": "CAMSAP3",
  "term_id": "GO:0003677",
  "term_label": "DNA binding"
}